{
  "gene": "UniProtKB:P20336",
  "gene_name": "Ras-related protein Rab-3A",
  "term_id": "GO:0008021",
  "term_label": "synaptic vesicle",
  "gene_symbol": "RAB3A"
}